{
  "term_id": "GO:0042178",
  "gene_symbol": "CYP2C18",
  "gene": "UniProtKB:P33260",
  "gene_name": "Cytochrome P450 2C18",
  "term_label": "xenobiotic catabolic process"
}